lactam metabolic process [GO:0072338] (biological process) Definition: The chemical reactions and pathways involving lactams, any cyclic amides of amino carboxylic acids, having a 1-azacycloalkan-2-one structure, or analogues having unsaturation or heteroatoms replacing one or more carbon atoms of the ring. Relationships: is a type of amide metabolic process [GO:0043603]; is a type of small molecule metabolic process [GO:0044281] Also known as: cellular lactam metabolic process, cellular lactam metabolism Subtypes: penicillin metabolic process [GO:0042316], creatinine metabolic process [GO:0046449], lactam biosynthetic process [GO:0072339], lactam catabolic process [GO:0072340], cephalosporin C metabolic process [GO:1901266] Sources: GOC:mah